chlorophyll cycle [GO:0033354] (biological process) Definition: A cyclic series of interconversions involving chlorophyll a, chlorophyll b and several chlorophyllide intermediates. Sources: GOC:mah, MetaCyc:PWY-5068 Relationships: is a type of chlorophyll metabolic process [GO:0015994]